{
  "term_id": "GO:0034236",
  "gene_symbol": "PRKAR2A",
  "term_label": "protein kinase A catalytic subunit binding",
  "gene_name": "cAMP-dependent protein kinase type II-alpha regulatory subunit",
  "gene": "UniProtKB:P13861"
}